{
  "term_id": "UNKNOWN:0001",
  "gene_name": "Putative uncharacterized protein SERTAD4-AS1",
  "gene_symbol": "SERTAD4-AS1",
  "term_label": "Unknown molecular function",
  "gene": "UniProtKB:Q5TG53"
}